{
  "term_id": "GO:0035556",
  "gene": "UniProtKB:P01185",
  "gene_name": "Vasopressin-neurophysin 2-copeptin",
  "term_label": "intracellular signal transduction",
  "gene_symbol": "AVP"
}